{
  "gene_symbol": "HDAC8",
  "gene_name": "Histone deacetylase 8",
  "term_id": "GO:0031507",
  "term_label": "heterochromatin formation",
  "gene": "UniProtKB:Q9BY41"
}